female meiotic nuclear division [GO:0007143] (biological process) Definition: A cell cycle process by which the cell nucleus divides as part of a meiotic cell cycle in the female germline. Note: Note that female germ lines can be found in female or hermaphroditic organisms, so this term can be used to annotate gene products from hermaphrodites such as those of C. elegans. See also the biological process term 'meiotic nuclear division; GO:0140013'. Sources: GOC:dph, GOC:ems, GOC:mah, GOC:vw Also known as: female meiosis, female meiotic division Relationships: is a type of meiotic nuclear division [GO:0140013]; is part of female gamete generation [GO:0007292] Subtypes: GO:0007144, GO:0007147